dTDP-4-dehydrorhamnose 3,5-epimerase activity [GO:0008830] (MF) Sources: EC:5.1.3.13, RHEA:16969 Definition: Catalysis of the reaction: dTDP-4-dehydro-6-deoxy-alpha-D-glucose = dTDP-4-dehydro-6-deoxy-L-mannose. Relationships: is a type of racemase and epimerase activity, acting on carbohydrates and derivatives [GO:0016857] Also known as: TDP-4-keto-L-rhamnose-3,5-epimerase activity, TDP-4-ketorhamnose 3,5-epimerase activity, dTDP-4-dehydro-6-deoxy-D-glucose 3,5-epimerase activity, dTDP-4-keto-6-deoxyglucose 3,5-epimerase activity, thymidine diphospho-4-ketorhamnose 3,5-epimerase activity